{
  "term_id": "UNKNOWN:0002",
  "gene_name": "Protein YIPF1",
  "gene_symbol": "YIPF1",
  "gene": "UniProtKB:Q9Y548",
  "term_label": "Unknown biological process"
}